{
  "gene": "UniProtKB:Q04725",
  "gene_name": "Transducin-like enhancer protein 2",
  "term_label": "transcription regulator complex",
  "term_id": "GO:0005667",
  "gene_symbol": "TLE2"
}